{
  "gene": "UniProtKB:Q9H1H9",
  "term_label": "microtubule motor activity",
  "gene_name": "Kinesin-like protein KIF13A",
  "gene_symbol": "KIF13A",
  "term_id": "GO:0003777"
}